{
  "gene_name": "Ran guanine nucleotide release factor",
  "gene": "UniProtKB:Q9HD47",
  "term_label": "heart contraction",
  "term_id": "GO:0060047",
  "gene_symbol": "RANGRF"
}